{
  "term_label": "Unknown cellular component",
  "gene_symbol": "IGHV3-21",
  "gene": "UniProtKB:A0A0B4J1V1",
  "gene_name": "Immunoglobulin heavy variable 3-21",
  "term_id": "UNKNOWN:0003"
}